{
  "gene": "UniProtKB:A8MRT5",
  "term_label": "Unknown cellular component",
  "term_id": "UNKNOWN:0003",
  "gene_name": "Nuclear pore complex-interacting protein family member B5",
  "gene_symbol": "NPIPB5"
}